{
  "term_label": "positive regulation of T cell activation",
  "gene_symbol": "HLA-DPB1",
  "gene_name": "HLA class II histocompatibility antigen, DP beta 1 chain",
  "gene": "UniProtKB:P04440",
  "term_id": "GO:0050870"
}